{
  "gene_symbol": "RPL11",
  "gene": "UniProtKB:P62913",
  "term_label": "structural constituent of ribosome",
  "gene_name": "Large ribosomal subunit protein uL5",
  "term_id": "GO:0003735"
}